ureteric peristalsis [GO:0072105] (biological process) Definition: A wavelike sequence of involuntary muscular contraction and relaxation that passes along the ureter, impelling the contents onwards. The ureter is one of a pair of thick-walled tubes that transports urine from the kidney pelvis to the urinary bladder. Sources: GOC:mtg_kidney_jan10 Relationships: is a type of ureter smooth muscle contraction [GO:0014849]; is a type of peristalsis [GO:0030432]